{
  "term_id": "GO:0010833",
  "gene": "UniProtKB:Q9NYB0",
  "gene_name": "Telomeric repeat-binding factor 2-interacting protein 1",
  "term_label": "telomere maintenance via telomere lengthening",
  "gene_symbol": "TERF2IP"
}